{
  "gene": "UniProtKB:Q8IVI9",
  "gene_name": "Nostrin",
  "gene_symbol": "NOSTRIN",
  "term_label": "Unknown cellular component",
  "term_id": "UNKNOWN:0003"
}